{
  "term_id": "UNKNOWN:0002",
  "gene_name": "Cleavage stimulation factor subunit 2 tau variant",
  "gene_symbol": "CSTF2T",
  "term_label": "Unknown biological process",
  "gene": "UniProtKB:Q9H0L4"
}